{
  "term_label": "Unknown molecular function",
  "gene_name": "Putative inactivation escape 1 protein",
  "gene": "UniProtKB:O15225",
  "term_id": "UNKNOWN:0001",
  "gene_symbol": "INE1"
}